{
  "gene": "UniProtKB:Q8WZ19",
  "gene_symbol": "KCTD13",
  "gene_name": "BTB_POZ domain-containing adapter for CUL3-mediated RhoA degradation protein 1",
  "term_label": "protein ubiquitination",
  "term_id": "GO:0016567"
}